{
  "term_id": "GO:0005886",
  "gene_name": "Puratrophin-1",
  "term_label": "plasma membrane",
  "gene_symbol": "PLEKHG4",
  "gene": "UniProtKB:Q58EX7"
}